{
  "gene_name": "Ral guanine nucleotide dissociation stimulator",
  "gene": "UniProtKB:Q12967",
  "term_id": "GO:0005886",
  "term_label": "plasma membrane",
  "gene_symbol": "RALGDS"
}